{
  "gene": "UniProtKB:P01706",
  "term_id": "UNKNOWN:0001",
  "gene_name": "Immunoglobulin lambda variable 2-11",
  "gene_symbol": "IGLV2-11",
  "term_label": "Unknown molecular function"
}